{
  "gene": "UniProtKB:P39023",
  "gene_symbol": "RPL3",
  "gene_name": "Large ribosomal subunit protein uL3",
  "term_label": "translation",
  "term_id": "GO:0006412"
}